{
  "gene_symbol": "NFIL3",
  "gene": "UniProtKB:Q16649",
  "gene_name": "Nuclear factor interleukin-3-regulated protein",
  "term_label": "circadian rhythm",
  "term_id": "GO:0007623"
}